{
  "term_label": "Unknown molecular function",
  "gene_symbol": "CYP4F3",
  "gene": "UniProtKB:Q08477",
  "gene_name": "Cytochrome P450 4F3",
  "term_id": "UNKNOWN:0001"
}